{
  "gene_symbol": "WRN",
  "term_id": "GO:0043138",
  "term_label": "3'-5' DNA helicase activity",
  "gene_name": "Bifunctional 3'-5' exonuclease_ATP-dependent helicase WRN",
  "gene": "UniProtKB:Q14191"
}